{
  "term_label": "Unknown biological process",
  "gene_name": "Lysosomal membrane ascorbate-dependent ferrireductase CYB561A3",
  "gene_symbol": "CYB561A3",
  "term_id": "UNKNOWN:0002",
  "gene": "UniProtKB:Q8NBI2"
}